humanin receptor complex [GO:7770013] (cellular component) Also known as: HN receptor complex Definition: A protein complex that acts as a receptor for the neuroprotective peptide humanin (HN). In humans the receptor complex is a trimer composed of CNTFR, IL6ST and IL27RA. HN binding to IL27RA and CNTFR induces oligomerization of the three subunits. References: PMID:19386761 Relationships: is a type of GO:0098802